{
  "gene_symbol": "TAOK1",
  "gene_name": "Serine_threonine-protein kinase TAO1",
  "term_label": "protein serine/threonine kinase activity",
  "gene": "UniProtKB:Q7L7X3",
  "term_id": "GO:0004674"
}